GMP catabolic process to guanine [GO:0006202] (biological process) Sources: ISBN:0198506732 Relationships: is a type of GMP catabolic process [GO:0046038]; is a type of guanine metabolic process [GO:0046098] Definition: The chemical reactions and pathways resulting in the breakdown of guanosine monophosphate into other compounds, including guanine. Also known as: GMP breakdown to guanine, GMP degradation to guanine